{
  "term_id": "GO:0030198",
  "gene_name": "A disintegrin and metalloproteinase with thrombospondin motifs 20",
  "term_label": "extracellular matrix organization",
  "gene": "UniProtKB:P59510",
  "gene_symbol": "ADAMTS20"
}